homodimeric polyprenyl diphosphate synthase complex [GO:0032477] (cellular component) Relationships: is a type of GO:0032476; is part of cytoplasm [GO:0005737] Also known as: homodimeric decaprenyl diphosphate synthase complex Definition: A homodimeric complex that possesses polyprenyl diphosphate synthase activity involved in the synthesis of the isoprenoid chain of ubiquinone whose length varies between organisms. References: PMID:14519123